photosystem II assembly [GO:0010207] (biological process) Relationships: is a type of protein-containing complex assembly [GO:0065003]; is part of photosynthesis, light reaction [GO:0019684] Sources: GOC:aa, GOC:pz Subtypes: GO:0010270 Definition: The aggregation, arrangement and bonding together of a set of components to form a photosystem II complex on the thylakoid membrane. The photosystem II complex consists of at least 20 polypeptides and around 80 cofactors in most organisms.